{
  "gene_symbol": "PRKCB",
  "term_id": "GO:0004674",
  "gene_name": "Protein kinase C beta type",
  "term_label": "protein serine/threonine kinase activity",
  "gene": "UniProtKB:P05771"
}